germ tube formation [GO:0075009] (BP) Definition: Development of slender tubular outgrowth first produced by most symbiont spores immediately following germination on or near its host organism. The host is defined as the larger of the organisms involved in a symbiotic interaction. Sources: GOC:pamgo_curators Also known as: germ tube formation on or near host Relationships: is a type of anatomical structure development [GO:0048856]; is part of GO:0009847 Regulation: RO_0002211 by regulation of germ tube formation [GO:0075010]; positively regulated by positive regulation of germ tube formation [GO:0075011]; RO_0002212 by negative regulation of germ tube formation [GO:0075012]